chromate transport [GO:0015703] (biological process) Relationships: is a type of GO:0015698 Sources: GOC:krc Definition: The directed movement of chromate into, out of or within a cell, or between cells, by means of some agent such as a transporter or pore.